{
  "gene_name": "Adenosine 5'-monophosphoramidase HINT2",
  "gene": "UniProtKB:Q9BX68",
  "term_id": "GO:0016787",
  "gene_symbol": "HINT2",
  "term_label": "hydrolase activity"
}